{
  "gene_symbol": "COL2A1",
  "term_id": "GO:0031012",
  "term_label": "extracellular matrix",
  "gene": "UniProtKB:P02458",
  "gene_name": "Collagen alpha-1(II) chain"
}